regulation of interleukin-12 production [GO:0032655] (biological process) Relationships: is a type of GO:0001817; regulates interleukin-12 production [GO:0032615] Also known as: regulation of IL-12 production, regulation of interleukin-12 biosynthetic process, regulation of interleukin-12 secretion, regulation of CLMF production, regulation of NKSF production Definition: Any process that modulates the frequency, rate, or extent of interleukin-12 production. Sources: GOC:mah Subtypes: GO:0032695, positive regulation of interleukin-12 production [GO:0032735]